{
  "term_id": "UNKNOWN:0001",
  "gene_symbol": "NT5C3B",
  "term_label": "Unknown molecular function",
  "gene_name": "7-methylguanosine phosphate-specific 5'-nucleotidase",
  "gene": "UniProtKB:Q969T7"
}